{
  "gene_name": "POTE ankyrin domain family member F",
  "gene": "UniProtKB:A5A3E0",
  "gene_symbol": "POTEF",
  "term_id": "GO:0035267",
  "term_label": "NuA4 histone acetyltransferase complex"
}